{
  "term_id": "UNKNOWN:0002",
  "gene": "UniProtKB:Q9H094",
  "gene_symbol": "NBPF3",
  "term_label": "Unknown biological process",
  "gene_name": "Neuroblastoma breakpoint family member 3"
}